{
  "term_label": "embryonic skeletal system development",
  "gene": "UniProtKB:P56179",
  "term_id": "GO:0048706",
  "gene_symbol": "DLX6",
  "gene_name": "Homeobox protein DLX-6"
}